regulation of Rab protein signal transduction [GO:0032483] (biological process) Definition: Any process that modulates the frequency, rate or extent of Rab protein signal transduction. Sources: GOC:mah Relationships: is a type of regulation of small GTPase mediated signal transduction [GO:0051056]; regulates Rab protein signal transduction [GO:0032482]